{
  "term_id": "GO:0016592",
  "gene_name": "Mediator of RNA polymerase II transcription subunit 13",
  "gene_symbol": "MED13",
  "term_label": "mediator complex",
  "gene": "UniProtKB:Q9UHV7"
}